myosin XIV complex [GO:0031484] (CC) References: PMID:10722873 Relationships: is a type of GO:0016461 Definition: A myosin complex containing a class XIV myosin heavy chain and associated light chains; myosin XIV heavy chains are the simplest known, containing a motor domain, no classic IQ motif and variable length tails.